{
  "gene_name": "HMG domain-containing protein 4",
  "term_label": "Unknown biological process",
  "term_id": "UNKNOWN:0002",
  "gene_symbol": "HMGXB4",
  "gene": "UniProtKB:Q9UGU5"
}